arsenate reductase (glutaredoxin) activity [GO:0008794] (molecular function) Definition: Catalysis of the reaction: arsenate + reduced glutaredoxin = arsenite + oxidized glutaredoxin. Glutaredoxin functions as the electron donor for arsenate reduction. The electron flow therefore is ( NADPH -> glutathione reductase (EC:1.6.4.2) -> ) glutathione -> glutaredoxin -> arsenate reductase, i.e. glutathione is reduced by glutathione reductase and glutaredoxin is reduced by glutathione. References: PMID:10593884 Sources: EC:1.20.4.1, GOC:kd Also known as: glutharedoxin:arsenate oxidoreductase activity Relationships: is a type of GO:0030614